{
  "gene_name": "Synemin",
  "gene_symbol": "SYNM",
  "term_label": "costamere",
  "term_id": "GO:0043034",
  "gene": "UniProtKB:O15061"
}